{
  "gene_symbol": "PPCDC",
  "gene_name": "Phosphopantothenoylcysteine decarboxylase",
  "term_id": "GO:0015937",
  "term_label": "coenzyme A biosynthetic process",
  "gene": "UniProtKB:Q96CD2"
}